{
  "gene": "UniProtKB:Q96Q89",
  "gene_symbol": "KIF20B",
  "term_id": "GO:0008017",
  "gene_name": "Kinesin-like protein KIF20B",
  "term_label": "microtubule binding"
}